{
  "term_id": "GO:1904121",
  "gene_symbol": "PLTP",
  "gene_name": "Phospholipid transfer protein",
  "gene": "UniProtKB:P55058",
  "term_label": "phosphatidylethanolamine transfer activity"
}